{
  "term_id": "GO:0005759",
  "gene_name": "FAST kinase domain-containing protein 3, mitochondrial",
  "gene_symbol": "FASTKD3",
  "gene": "UniProtKB:Q14CZ7",
  "term_label": "mitochondrial matrix"
}